{
  "gene": "UniProtKB:P60985",
  "gene_symbol": "KRTDAP",
  "term_id": "GO:0005615",
  "term_label": "extracellular space",
  "gene_name": "Keratinocyte differentiation-associated protein"
}